{
  "gene_symbol": "TDO2",
  "gene_name": "Tryptophan 2,3-dioxygenase",
  "gene": "UniProtKB:P48775",
  "term_id": "GO:0004833",
  "term_label": "L-tryptophan 2,3-dioxygenase activity"
}